regulation of endoplasmic reticulum tubular network organization [GO:1903371] (biological process) References: PMID:24891604 Sources: GOC:TermGenie, GOC:als, GO_REF:0000058 Definition: Any process that modulates the frequency, rate or extent of endoplasmic reticulum tubular network organization. Subtypes: GO:1903372, positive regulation of endoplasmic reticulum tubular network organization [GO:1903373] Relationships: is a type of regulation of organelle organization [GO:0033043]; regulates GO:0071786 Also known as: regulation of ER tubular network organisation, regulation of ER tubular network organization, regulation of endoplasmic reticulum tubular network organisation